{
  "gene": "UniProtKB:O75385",
  "gene_symbol": "ULK1",
  "gene_name": "Serine_threonine-protein kinase ULK1",
  "term_label": "autophagosome",
  "term_id": "GO:0005776"
}